uterine smooth muscle contraction [GO:0070471] (BP) Regulation: regulated by regulation of uterine smooth muscle contraction [GO:0070472]; negatively regulated by GO:0070473; positively regulated by positive regulation of uterine smooth muscle contraction [GO:0070474] Sources: GOC:sl Relationships: is a type of smooth muscle contraction [GO:0006939] Definition: A process in which force is generated within smooth muscle tissue, resulting in a change in muscle geometry. This process occurs in the uterus. Force generation involves a chemo-mechanical energy conversion step that is carried out by the actin/myosin complex activity, which generates force through ATP hydrolysis. The uterus is a muscular organ of the female mammal for containing and usually for nourishing the young during development prior to birth. Also known as: myometrial contraction, myometrial smooth muscle contraction, myometrium contraction